{
  "term_id": "GO:0006108",
  "term_label": "malate metabolic process",
  "gene_symbol": "ME1",
  "gene_name": "NADP-dependent malic enzyme",
  "gene": "UniProtKB:P48163"
}